{
  "gene": "UniProtKB:Q9HB89",
  "term_id": "GO:0008188",
  "gene_name": "Neuromedin-U receptor 1",
  "term_label": "neuropeptide receptor activity",
  "gene_symbol": "NMUR1"
}